{
  "term_label": "endosome membrane",
  "gene": "UniProtKB:Q8N2U9",
  "gene_symbol": "SLC66A2",
  "term_id": "GO:0010008",
  "gene_name": "Solute carrier family 66 member 2"
}